benzoate catabolic process via CoA ligation [GO:0010128] (biological process) Relationships: is a type of benzoate catabolic process [GO:0043639] Sources: GOC:pz Definition: The chemical reactions and pathways resulting in the breakdown of benzoate, by its ligation to Coenzyme A to form benzoyl-CoA, which is then broken by an aerobic or anaerobic pathway. Also known as: anaerobic benzoate breakdown, anaerobic benzoate catabolic process, anaerobic benzoate catabolism, anaerobic benzoate degradation